{
  "gene": "UniProtKB:Q9UF83",
  "gene_name": "Uncharacterized protein DKFZp434B061",
  "term_id": "UNKNOWN:0003",
  "gene_symbol": "Q9UF83",
  "term_label": "Unknown cellular component"
}